{
  "gene_name": "DnaJ homolog subfamily A member 2",
  "gene": "UniProtKB:O60884",
  "term_label": "ATPase activator activity",
  "term_id": "GO:0001671",
  "gene_symbol": "DNAJA2"
}